{
  "term_label": "cell differentiation involved in embryonic placenta development",
  "gene_name": "Chorion-specific transcription factor GCMa",
  "gene": "UniProtKB:Q9NP62",
  "gene_symbol": "GCM1",
  "term_id": "GO:0060706"
}